{
  "gene_name": "MHC class I polypeptide-related sequence B",
  "gene": "UniProtKB:Q29980",
  "term_id": "GO:0046629",
  "gene_symbol": "MICB",
  "term_label": "gamma-delta T cell activation"
}